response to biphenyl [GO:1904614] (biological process) Definition: Any process that results in a change in state or activity of a cell or an organism (in terms of movement, secretion, enzyme production, gene expression, etc.) as a result of a biphenyl stimulus. References: PMID:23196670 Sources: GOC:TermGenie, GO_REF:0000071 Relationships: is a type of GO:0042221 Subtypes: cellular response to biphenyl [GO:1904615]